{
  "term_label": "mitochondrion",
  "gene": "UniProtKB:Q9Y291",
  "term_id": "GO:0005739",
  "gene_symbol": "MRPS33",
  "gene_name": "Small ribosomal subunit protein mS33"
}